{
  "term_id": "GO:0019901",
  "term_label": "protein kinase binding",
  "gene_name": "5'-AMP-activated protein kinase subunit beta-2",
  "gene": "UniProtKB:O43741",
  "gene_symbol": "PRKAB2"
}